proctolin receptor activity [GO:0035236] (molecular function) Sources: GOC:bf Relationships: is a type of GO:0008188 Definition: Combining with the neuropeptide proctolin, to initiate a change in cell activity.